{
  "gene_name": "Importin subunit alpha-4",
  "gene": "UniProtKB:O00505",
  "term_label": "NLS-bearing protein import into nucleus",
  "gene_symbol": "KPNA3",
  "term_id": "GO:0006607"
}